{
  "term_id": "GO:0016020",
  "gene_name": "Potassium voltage-gated channel subfamily S member 1",
  "term_label": "membrane",
  "gene_symbol": "KCNS1",
  "gene": "UniProtKB:Q96KK3"
}